{
  "term_label": "molecular adaptor activity",
  "gene_name": "Axin-1",
  "gene": "UniProtKB:O15169",
  "gene_symbol": "AXIN1",
  "term_id": "GO:0060090"
}